{
  "gene_name": "Argininosuccinate synthase",
  "gene_symbol": "ASS1",
  "term_id": "GO:0005737",
  "gene": "UniProtKB:P00966",
  "term_label": "cytoplasm"
}